positive regulation of semaphorin-plexin signaling pathway [GO:2001262] (biological process) Sources: GOC:BHF Also known as: positive regulation of semaphorin-plexin signalling pathway Definition: Any process that activates or increases the frequency, rate or extent of semaphorin-plexin signaling pathway. Relationships: is a type of positive regulation of signal transduction [GO:0009967]; is_a regulation of semaphorin-plexin signaling pathway [GO:2001260]; positively regulates semaphorin-plexin signaling pathway [GO:0071526] Subtypes: GO:2000764